intracellular nucleotide homeostasis [GO:0140979] (BP) Relationships: is a type of intracellular chemical homeostasis [GO:0055082] References: PMID:23416111, PMID:34880500 Definition: A homeostatic process involved in the maintenance of a steady state level of nucleotides within a cell.